{
  "gene_symbol": "CYP4Z2P",
  "term_id": "UNKNOWN:0001",
  "gene_name": "Putative inactive cytochrome P450 family member 4Z2",
  "term_label": "Unknown molecular function",
  "gene": "UniProtKB:Q8N1L4"
}